{
  "term_label": "microtubule organizing center organization",
  "gene_name": "HAUS augmin-like complex subunit 3",
  "term_id": "GO:0031023",
  "gene": "UniProtKB:Q68CZ6",
  "gene_symbol": "HAUS3"
}